Golgi-associated vesicle lumen [GO:0070931] (cellular component) Relationships: is a type of cytoplasmic vesicle lumen [GO:0060205]; is part of Golgi apparatus [GO:0005794]; is part of GO:0005798 Sources: GOC:mah Definition: The volume enclosed by the membrane of a Golgi-associated vesicle.